{
  "gene_name": "Protein CBFA2T1",
  "gene": "UniProtKB:Q06455",
  "term_label": "negative regulation of DNA-templated transcription",
  "gene_symbol": "RUNX1T1",
  "term_id": "GO:0045892"
}